{
  "term_id": "UNKNOWN:0002",
  "gene": "UniProtKB:O95944",
  "gene_symbol": "NCR2",
  "term_label": "Unknown biological process",
  "gene_name": "Natural cytotoxicity triggering receptor 2"
}